{
  "term_label": "ephrin receptor binding",
  "gene_name": "Ankyrin repeat and sterile alpha motif domain-containing protein 1B",
  "gene": "UniProtKB:Q7Z6G8",
  "term_id": "GO:0046875",
  "gene_symbol": "ANKS1B"
}